{
  "term_id": "GO:0046339",
  "term_label": "diacylglycerol metabolic process",
  "gene_name": "Diacylglycerol O-acyltransferase 2",
  "gene_symbol": "DGAT2",
  "gene": "UniProtKB:Q96PD7"
}